{
  "term_id": "GO:0007189",
  "gene_symbol": "MC5R",
  "term_label": "adenylate cyclase-activating G protein-coupled receptor signaling pathway",
  "gene": "UniProtKB:P33032",
  "gene_name": "Melanocortin receptor 5"
}